positive regulation of sodium ion transport [GO:0010765] (biological process) Subtypes: positive regulation of sodium ion transmembrane transport [GO:1902307] Relationships: is a type of regulation of sodium ion transport [GO:0002028]; is a type of positive regulation of monoatomic ion transport [GO:0043270]; positively regulates sodium ion transport [GO:0006814] Definition: Any process that increases the frequency, rate or extent of the directed movement of sodium ions (Na+) into, out of or within a cell, or between cells, by means of some agent such as a transporter or pore. Sources: GOC:dph, GOC:tb